{
  "term_id": "GO:0007601",
  "gene": "UniProtKB:Q8WXF5",
  "gene_symbol": "CRYGN",
  "gene_name": "Gamma-crystallin N",
  "term_label": "visual perception"
}